{
  "gene_name": "Protein tyrosine phosphatase type IVA 2",
  "gene_symbol": "PTP4A2",
  "term_id": "GO:0005737",
  "term_label": "cytoplasm",
  "gene": "UniProtKB:Q12974"
}